{
  "term_id": "GO:0005634",
  "gene_name": "Nucleolar transcription factor 1",
  "term_label": "nucleus",
  "gene_symbol": "UBTF",
  "gene": "UniProtKB:P17480"
}